L-ascorbate:sodium symporter activity [GO:0008520] (molecular function) References: PMID:18094143 Sources: GOC:mah, GOC:yaf Definition: Enables the transfer of a solute or solutes from one side of a membrane to the other according to the reaction: L-ascorbate(out) + Na+(out) = L-ascorbate(in) + Na+(in). Relationships: is a type of organic acid:sodium symporter activity [GO:0005343]; is a type of carbohydrate:monoatomic cation symporter activity [GO:0005402]; is a type of monosaccharide transmembrane transporter activity [GO:0015145]; is a type of carboxylic acid transmembrane transporter activity [GO:0046943] Also known as: sodium-dependent L-ascorbate transmembrane transporter activity, sodium-dependent L-ascorbic acid transporter